{
  "gene_name": "Probable inactive 1-aminocyclopropane-1-carboxylate synthase-like protein 2",
  "gene": "UniProtKB:Q4AC99",
  "term_id": "GO:0008483",
  "term_label": "transaminase activity",
  "gene_symbol": "ACCSL"
}